alpha3-beta1 integrin-CD151 complex [GO:0071058] (cellular component) Definition: A protein complex that consists of an alpha3-beta1 integrin complex bound to the tetraspanin CD151. References: PMID:10811835, PMID:11884516 Relationships: is a type of plasma membrane protein complex [GO:0098797] Also known as: ITGA3-ITGB1-CD151 complex